{
  "gene_symbol": "ELOVL4",
  "gene_name": "Elongation of very long chain fatty acids protein 4",
  "term_id": "GO:0005789",
  "gene": "UniProtKB:Q9GZR5",
  "term_label": "endoplasmic reticulum membrane"
}